response to cordycepin [GO:1904309] (BP) Also known as: response to 3'-deoxyadenosine Subtypes: GO:1904310 References: PMID:21597460 Sources: GOC:TermGenie, GO_REF:0000071 Definition: Any process that results in a change in state or activity of a cell or an organism (in terms of movement, secretion, enzyme production, gene expression, etc.) as a result of a cordycepin stimulus. Relationships: is a type of response to purine-containing compound [GO:0014074]; is a type of GO:1901700